{
  "gene": "UniProtKB:Q9Y5H5",
  "gene_symbol": "PCDHA9",
  "gene_name": "Protocadherin alpha-9",
  "term_label": "cell adhesion",
  "term_id": "GO:0007155"
}